{
  "gene_name": "Tumor suppressor candidate gene 1 protein",
  "gene_symbol": "TUSC1",
  "term_id": "UNKNOWN:0003",
  "gene": "UniProtKB:Q2TAM9",
  "term_label": "Unknown cellular component"
}